{
  "gene_symbol": "CD74",
  "gene_name": "HLA class II histocompatibility antigen gamma chain",
  "term_label": "cytoplasm",
  "gene": "UniProtKB:P04233",
  "term_id": "GO:0005737"
}